proteasomal proteolysis associated with antigen processing and presentation [GO:0002497] (biological process) Definition: The hydrolysis of a peptide bond or bonds within a protein by the proteasome complex contributing to antigen processing and presentation. References: PMID:15224092, PMID:15771591 Sources: GOC:add, ISBN:0781735149 Relationships: is a type of proteolysis associated with antigen processing and presentation [GO:0002496]